anaerobic respiration, using ammonium as electron donor [GO:0019331] (biological process) Definition: The oxidation of ammonium (NH4) to nitrogen (N2) in the absence of oxygen, using nitrite (NO2) as the electron acceptor. Hydroxylamine and ammonium are combined to yield hydrazine, which is subsequently oxidized to N2. Relationships: is a type of GO:0009061; is a type of energy derivation by oxidation of reduced inorganic compounds [GO:0015975]; is a type of ammonia oxidation [GO:0019329]; is a type of nitrogen cycle metabolic process [GO:0071941] Also known as: ammonia oxidation, anaerobic ammonium oxidation, anammox Sources: MetaCyc:P303-PWY